{
  "gene_name": "Solute carrier family 2, facilitated glucose transporter member 4",
  "term_id": "GO:0005886",
  "gene_symbol": "SLC2A4",
  "gene": "UniProtKB:P14672",
  "term_label": "plasma membrane"
}